negative regulation of translational elongation [GO:0045900] (biological process) Relationships: is a type of GO:0006448; is_a GO:0017148; negatively regulates translational elongation [GO:0006414] Also known as: down regulation of translational elongation, down-regulation of translational elongation, downregulation of translational elongation, inhibition of translational elongation Sources: GOC:go_curators Definition: Any process that stops, prevents, or reduces the frequency, rate or extent of translational elongation. Subtypes: negative regulation of cytoplasmic translational elongation [GO:1900248], GO:1904570, GO:1905083, GO:2001125